{
  "gene": "UniProtKB:P35462",
  "term_label": "regulation of potassium ion transport",
  "term_id": "GO:0043266",
  "gene_symbol": "DRD3",
  "gene_name": "D(3) dopamine receptor"
}